{
  "term_id": "GO:0060271",
  "gene": "UniProtKB:Q9BYV8",
  "term_label": "cilium assembly",
  "gene_name": "Centrosomal protein of 41 kDa",
  "gene_symbol": "CEP41"
}